{
  "term_id": "GO:0005886",
  "gene": "UniProtKB:Q9NRW4",
  "gene_name": "Dual specificity protein phosphatase 22",
  "gene_symbol": "DUSP22",
  "term_label": "plasma membrane"
}